SA node cell-atrial cardiac muscle cell adhesion involved in cell communication [GO:0086022] (biological process) Sources: GOC:BHF, GOC:mtg_cardiac_conduct_nov11 Also known as: SA cardiac muscle cell-atrial cardiac muscle cell adhesion involved in cell communication, SA cardiomyocyte-atrial cardiomyocyte adhesion involved in cell communication, SAN cardiomyocyte-atrial cardiomyocyte adhesion involved in cell communication, sinoatrial node cardiomyocyte-atrial cardiomyocyte adhesion involved in cell communication, sinus node cardiomyocyte-atrial cardiomyocyte adhesion involved in cell communication Relationships: is a type of heterotypic cell-cell adhesion [GO:0034113]; is a type of GO:0086042; is part of SA node cell to atrial cardiac muscle cell communication [GO:0086070] Definition: The attachment of SA node cardiomyocyte to an atrial cardiomyocyte via adhesion molecules that results in the cells being juxtaposed so that they can communicate.